{
  "term_label": "Unknown cellular component",
  "term_id": "UNKNOWN:0003",
  "gene": "UniProtKB:Q8TAE6",
  "gene_name": "Protein phosphatase 1 regulatory subunit 14C",
  "gene_symbol": "PPP1R14C"
}